{
  "gene_symbol": "MRPS18B",
  "term_id": "GO:0005763",
  "gene": "UniProtKB:Q9Y676",
  "term_label": "mitochondrial small ribosomal subunit",
  "gene_name": "Small ribosomal subunit protein mS40"
}